{
  "gene_symbol": "OR8B4",
  "term_id": "GO:0004984",
  "term_label": "olfactory receptor activity",
  "gene_name": "Olfactory receptor 8B4",
  "gene": "UniProtKB:Q96RC9"
}